polytene chromosome [GO:0005700] (cellular component) Sources: ISBN:0198506732 Definition: A type of chromosome in a polyploid cell, formed when multiple copies of homologous chromosomes are aligned side by side to give a giant chromosome in which distinct chromosome bands are readily visible. Relationships: is a type of chromosome [GO:0005694]